{
  "gene": "UniProtKB:Q9BV47",
  "term_id": "GO:0005737",
  "gene_symbol": "DUSP26",
  "gene_name": "Dual specificity protein phosphatase 26",
  "term_label": "cytoplasm"
}